{
  "term_id": "UNKNOWN:0001",
  "gene_symbol": "ZMYND19",
  "term_label": "Unknown molecular function",
  "gene_name": "Zinc finger MYND domain-containing protein 19",
  "gene": "UniProtKB:Q96E35"
}